{
  "gene_name": "WD repeat-containing protein 97",
  "term_label": "Unknown molecular function",
  "gene_symbol": "WDR97",
  "term_id": "UNKNOWN:0001",
  "gene": "UniProtKB:A6NE52"
}